gentamycin biosynthetic process [GO:1901130] (BP) Definition: The chemical reactions and pathways resulting in the formation of gentamycin. Also known as: gentamycin anabolism, gentamycin biosynthesis, gentamycin formation, gentamycin synthesis Relationships: is a type of aminoglycoside antibiotic biosynthetic process [GO:0030648]; is_a polyol biosynthetic process [GO:0046173]; is a type of gentamycin metabolic process [GO:1901128] Sources: GOC:TermGenie, GOC:yaf, UniPathway:UPA00967